{
  "gene": "UniProtKB:Q96M69",
  "term_label": "GMP kinase activity",
  "term_id": "GO:0004385",
  "gene_name": "Leucine-rich repeat and guanylate kinase domain-containing protein",
  "gene_symbol": "LRGUK"
}